{
  "gene_symbol": "KCTD13",
  "gene": "UniProtKB:Q8WZ19",
  "term_id": "GO:0031463",
  "term_label": "Cul3-RING ubiquitin ligase complex",
  "gene_name": "BTB_POZ domain-containing adapter for CUL3-mediated RhoA degradation protein 1"
}